D-arabinitol 2-dehydrogenase activity [GO:0047038] (molecular function) Definition: Catalysis of the reaction: D-arabinitol + NAD+ = D-ribulose + H+ + NADH. Sources: EC:1.1.1.250, RHEA:17389 Also known as: D-arabinitol 2-dehydrogenase (ribulose-forming) activity, D-arabinitol:NAD+ 2-oxidoreductase (D-ribulose-forming) Relationships: is a type of GO:0016616